{
  "gene_symbol": "ST8SIA2",
  "gene": "UniProtKB:Q92186",
  "term_id": "GO:0006491",
  "gene_name": "Alpha-2,8-sialyltransferase 8B",
  "term_label": "N-glycan processing"
}